{
  "gene_name": "T cell receptor delta joining 4 (Fragment)",
  "term_id": "UNKNOWN:0001",
  "term_label": "Unknown molecular function",
  "gene_symbol": "TRDJ4",
  "gene": "UniProtKB:A0A075B6Z4"
}